protein N-acetylglucosaminyltransferase activity [GO:0016262] (molecular function) Also known as: UDP-N-acetyl-D-glucosamine:protein beta-N-acetyl-D-glucosaminyl-transferase activity, UDP-N-acetylglucosamine-peptide N-acetylglucosaminyltransferase activity, protein N-GlcNAc transferase activity, uridine diphospho-N-acetylglucosamine:polypeptide beta-N-acetylglucosaminyltransferase activity, uridine diphosphoacetylglucosamine-protein acetylglucosaminyltransferase activity, N-GlcNAc transferase activity Sources: EC:2.4.1.94 Subtypes: protein-arginine N-acetylglucosaminyltransferase activity [GO:0106362] Relationships: is a type of GO:0008375; is a type of catalytic activity, acting on a protein [GO:0140096] Definition: Catalysis of the reaction: UDP-N-acetyl-D-glucosamine + protein = UDP + 4-N-(N-acetyl-D-glucosaminyl)-protein.